{
  "term_id": "GO:0007268",
  "gene": "UniProtKB:Q05586",
  "gene_name": "Glutamate receptor ionotropic, NMDA 1",
  "gene_symbol": "GRIN1",
  "term_label": "chemical synaptic transmission"
}